{
  "gene": "UniProtKB:Q9Y5K3",
  "gene_name": "Choline-phosphate cytidylyltransferase B",
  "gene_symbol": "PCYT1B",
  "term_id": "GO:0031210",
  "term_label": "phosphatidylcholine binding"
}